activator ecdysone receptor complex [GO:0008232] (cellular component) Relationships: is a type of ecdysone receptor holocomplex [GO:0008230] References: PMID:10488333 Also known as: activator ecdysone receptor holocomplex Definition: A protein complex consisting of a heterodimer of Ecdysone receptor (EcR) and ultraspiracle (usp) bound to the ligand ecdysone, which activates transcription of target genes.